{
  "gene": "UniProtKB:P32418",
  "gene_name": "Sodium_calcium exchanger 1",
  "term_id": "GO:0005432",
  "gene_symbol": "SLC8A1",
  "term_label": "calcium:sodium antiporter activity"
}